{
  "gene_symbol": "IWS1",
  "term_id": "GO:0016973",
  "gene": "UniProtKB:Q96ST2",
  "gene_name": "Protein IWS1 homolog",
  "term_label": "poly(A)+ mRNA export from nucleus"
}